condensed chromosome [GO:0000793] (cellular component) Relationships: is a type of chromosome [GO:0005694] Note: Note that this term can be used to annotate gene products that localize to a mitotic chromosome in an organism that undergoes an 'open mitosis' in which the nuclear envelope breaks down during mitosis. Subtypes: condensed nuclear chromosome [GO:0000794] Definition: A highly compacted molecule of DNA and associated proteins resulting in a cytologically distinct structure. Sources: GOC:elh Also known as: cytoplasmic mitotic chromosome, metaphase chromosome, mitotic chromosome